cholesterol biosynthetic process via 24,25-dihydrolanosterol [GO:0033488] (biological process) Definition: The chemical reactions and pathways resulting in the formation of cholesterol, cholest-5-en-3 beta-ol, via the intermediate 24,25-dihydrolanosterol. Sources: GOC:mah, MetaCyc:PWY66-3 Relationships: is a type of GO:0006695 Also known as: cholesterol anabolism via 24,25-dihydrolanosterol, cholesterol biosynthesis via 24,25-dihydrolanosterol, cholesterol formation via 24,25-dihydrolanosterol, cholesterol synthesis via 24,25-dihydrolanosterol